regulation of biosynthetic process of antibacterial peptides active against Gram-negative bacteria [GO:0002813] (biological process) Subtypes: negative regulation of biosynthetic process of antibacterial peptides active against Gram-negative bacteria [GO:0002814], positive regulation of biosynthetic process of antibacterial peptides active against Gram-negative bacteria [GO:0006964] Definition: Any process that modulates the frequency, rate, or extent of biosynthesis of antibacterial peptides active against Gram-negative bacteria. Relationships: is a type of regulation of antibacterial peptide biosynthetic process [GO:0002808]; regulates GO:0002812 Sources: GOC:add